{
  "gene_symbol": "DDR2",
  "gene": "UniProtKB:Q16832",
  "term_label": "cell surface receptor protein tyrosine kinase signaling pathway",
  "term_id": "GO:0007169",
  "gene_name": "Discoidin domain-containing receptor 2"
}